{
  "gene": "UniProtKB:P55010",
  "gene_name": "Eukaryotic translation initiation factor 5",
  "gene_symbol": "EIF5",
  "term_id": "GO:0071074",
  "term_label": "eukaryotic initiation factor eIF2 binding"
}